TPR domain binding [GO:0030911] (molecular function) Sources: GOC:mah Also known as: tetratricopeptide repeat domain binding Definition: Binding to a tetratricopeptide repeat (TPR) domain of a protein, the consensus sequence of which is defined by a pattern of small and large hydrophobic amino acids and a structure composed of helices. Relationships: is a type of protein domain specific binding [GO:0019904]